{
  "term_label": "T cell activation",
  "gene_symbol": "SLAMF7",
  "gene_name": "SLAM family member 7",
  "gene": "UniProtKB:Q9NQ25",
  "term_id": "GO:0042110"
}